{
  "term_id": "UNKNOWN:0001",
  "term_label": "Unknown molecular function",
  "gene": "UniProtKB:A0A1B0GTJ6",
  "gene_symbol": "LOC101059948",
  "gene_name": "HCG1796489"
}